{
  "term_label": "lysosomal membrane",
  "gene": "UniProtKB:P49281",
  "gene_name": "Natural resistance-associated macrophage protein 2",
  "gene_symbol": "SLC11A2",
  "term_id": "GO:0005765"
}